{
  "gene": "UniProtKB:Q9Y6X6",
  "gene_symbol": "MYO16",
  "term_id": "GO:2000134",
  "gene_name": "Unconventional myosin-XVI",
  "term_label": "negative regulation of G1/S transition of mitotic cell cycle"
}